id [oboInOwl#id]